{
  "term_id": "GO:0005634",
  "gene_name": "Zinc finger protein 607",
  "gene_symbol": "ZNF607",
  "gene": "UniProtKB:Q96SK3",
  "term_label": "nucleus"
}